regulation of ornithine metabolic process [GO:0090368] (biological process) Sources: GOC:dph, GOC:jp, GOC:tb Subtypes: regulation of ornithine catabolic process [GO:1903266] Relationships: is a type of regulation of amino acid metabolic process [GO:0006521]; is_a regulation of small molecule metabolic process [GO:0062012]; regulates ornithine metabolic process [GO:0006591] Definition: Any process that modulates the rate, frequency, or extent of the chemical reactions and pathways involving ornithine, an amino acid only rarely found in proteins, but which is important in living organisms as an intermediate in the reactions of the urea cycle and in arginine biosynthesis.